structural constituent of ascospore wall [GO:1990915] (MF) References: PMID:24623719 Relationships: is a type of GO:0005199; occurs in ascospore wall [GO:0005619] Definition: The action of a molecule that contributes to the structural integrity of an ascospore wall.